{
  "term_id": "GO:0000978",
  "gene": "UniProtKB:Q9UMR3",
  "gene_name": "T-box transcription factor TBX20",
  "term_label": "RNA polymerase II cis-regulatory region sequence-specific DNA binding",
  "gene_symbol": "TBX20"
}